{
  "term_id": "GO:0071035",
  "gene": "UniProtKB:Q9NQT5",
  "gene_symbol": "EXOSC3",
  "gene_name": "Exosome complex component RRP40",
  "term_label": "nuclear polyadenylation-dependent rRNA catabolic process"
}